{
  "gene_name": "Protein transport protein Sec23B",
  "gene": "UniProtKB:Q15437",
  "term_id": "GO:0005096",
  "term_label": "GTPase activator activity",
  "gene_symbol": "SEC23B"
}